{
  "term_label": "plasma membrane",
  "gene_name": "Pikachurin",
  "gene": "UniProtKB:Q63HQ2",
  "gene_symbol": "EGFLAM",
  "term_id": "GO:0005886"
}